{
  "gene_name": "Calsyntenin-3",
  "gene_symbol": "CLSTN3",
  "term_label": "positive regulation of synapse assembly",
  "term_id": "GO:0051965",
  "gene": "UniProtKB:Q9BQT9"
}